{
  "term_id": "GO:0043161",
  "term_label": "proteasome-mediated ubiquitin-dependent protein catabolic process",
  "gene_name": "PRAME family member 22",
  "gene_symbol": "PRAMEF22",
  "gene": "UniProtKB:A3QJZ6"
}